{
  "gene_name": "Early growth response protein 3",
  "gene": "UniProtKB:Q06889",
  "term_label": "DNA-binding transcription factor activity, RNA polymerase II-specific",
  "term_id": "GO:0000981",
  "gene_symbol": "EGR3"
}